{
  "gene_name": "Ankyrin repeat domain-containing protein 33B",
  "gene": "UniProtKB:A6NCL7",
  "gene_symbol": "ANKRD33B",
  "term_label": "Unknown molecular function",
  "term_id": "UNKNOWN:0001"
}